1,2-diacylglycerol 3-beta-galactosyltransferase activity [GO:0046509] (molecular function) Also known as: MGDG synthase activity, UDP galactose-1,2-diacylglycerol galactosyltransferase activity, UDP-galactose-diacylglyceride galactosyltransferase activity, UDP-galactose:diacylglycerol galactosyltransferase activity, monogalactosyldiacylglycerol synthase activity, uridine diphosphogalactose-1,2-diacylglycerol galactosyltransferase activity, 1-beta-MGDG activity, 1beta-MGDG, UDP-galactose:1,2-diacyl-sn-glycerol 3-beta-D-galactosyltransferase activity, UDPgalactose:1,2-diacylglycerol 3-beta-D-galactosyltransferase activity Sources: EC:2.4.1.46, RHEA:14945 Definition: Catalysis of the reaction: 1,2-diacyl-sn-glycerol + UDP-D-galactose = 1,2-diacyl-3-beta-D-galactosyl-sn-glycerol + H+ + UDP. Relationships: is a type of UDP-galactosyltransferase activity [GO:0035250]